{
  "term_id": "GO:0036159",
  "gene_name": "Dynein axonemal intermediate chain 3",
  "gene_symbol": "DNAI3",
  "gene": "UniProtKB:Q8IWG1",
  "term_label": "inner dynein arm assembly"
}